renal response to blood flow involved in circulatory renin-angiotensin regulation of systemic arterial blood pressure [GO:0001999] (biological process) Relationships: is a type of renal system process involved in regulation of systemic arterial blood pressure [GO:0003071]; is part of regulation of systemic arterial blood pressure by circulatory renin-angiotensin [GO:0001991] Definition: The physiological response of the kidneys to a decrease in blood flow. Sources: GOC:dph Also known as: renal response to blood flow during renin-angiotensin control of blood pressure